{
  "term_id": "GO:0008403",
  "gene_symbol": "CYP24A1",
  "gene_name": "1,25-dihydroxyvitamin D(3) 24-hydroxylase, mitochondrial",
  "term_label": "25-hydroxycholecalciferol-24-hydroxylase activity",
  "gene": "UniProtKB:Q07973"
}